{
  "gene_symbol": "ACAN",
  "term_id": "GO:0007417",
  "gene": "UniProtKB:P16112",
  "term_label": "central nervous system development",
  "gene_name": "Aggrecan core protein"
}